{
  "gene_symbol": "CALCB",
  "gene_name": "Calcitonin gene-related peptide 2",
  "term_label": "adenylate cyclase-activating G protein-coupled receptor signaling pathway",
  "gene": "UniProtKB:P10092",
  "term_id": "GO:0007189"
}